{
  "gene": "UniProtKB:Q6XUX3",
  "gene_name": "Dual serine_threonine and tyrosine protein kinase",
  "gene_symbol": "DSTYK",
  "term_id": "GO:0005737",
  "term_label": "cytoplasm"
}